{
  "term_id": "GO:0007094",
  "gene": "UniProtKB:O95229",
  "term_label": "mitotic spindle assembly checkpoint signaling",
  "gene_name": "ZW10 interactor",
  "gene_symbol": "ZWINT"
}